{
  "gene_symbol": "OSBPL10",
  "term_label": "Unknown biological process",
  "term_id": "UNKNOWN:0002",
  "gene": "UniProtKB:Q9BXB5",
  "gene_name": "Oxysterol-binding protein-related protein 10"
}